{
  "gene_symbol": "FAM223B",
  "gene": "UniProtKB:A6NKX1",
  "gene_name": "Protein FAM223B",
  "term_id": "UNKNOWN:0003",
  "term_label": "Unknown cellular component"
}